positive regulation of regulated secretory pathway [GO:1903307] (biological process) References: PMID:12526776 Sources: GOC:PARL, GOC:TermGenie, GOC:pad, GO_REF:0000058 Note: An example of this is protein domain-specific expression of Synaptotagmin 1 in rat (P21707) in PMID:12526776 inferred from mutant phenotype. Definition: Any process that activates or increases the frequency, rate or extent of regulated secretory pathway. Subtypes: GO:0043302, positive regulation of calcium ion-dependent exocytosis [GO:0045956], positive regulation of synaptic vesicle exocytosis [GO:2000302] Relationships: is a type of positive regulation of exocytosis [GO:0045921]; is a type of regulation of regulated secretory pathway [GO:1903305]; positively regulates regulated exocytosis [GO:0045055] Also known as: up regulation of regulated secretory pathway, up-regulation of regulated secretory pathway, upregulation of regulated secretory pathway, activation of regulated secretory pathway